{
  "gene_name": "Cullin-4B",
  "gene": "UniProtKB:Q13620",
  "term_label": "nucleus",
  "term_id": "GO:0005634",
  "gene_symbol": "CUL4B"
}